{
  "term_id": "GO:0005811",
  "term_label": "lipid droplet",
  "gene_name": "Lipid transferase CIDEC",
  "gene_symbol": "CIDEC",
  "gene": "UniProtKB:Q96AQ7"
}